{
  "gene_name": "LysM and putative peptidoglycan-binding domain-containing protein 1",
  "term_id": "UNKNOWN:0001",
  "term_label": "Unknown molecular function",
  "gene": "UniProtKB:Q96S90",
  "gene_symbol": "LYSMD1"
}